collagen type XVIII trimer [GO:0030938] (cellular component) References: PMID:21421911 Definition: A collagen homotrimer of alpha1(XVIII) chains. Relationships: is a type of multiplexin collagen trimer [GO:0140156]